{
  "gene": "UniProtKB:Q6GMV3",
  "gene_symbol": "PTRHD1",
  "term_id": "UNKNOWN:0001",
  "term_label": "Unknown molecular function",
  "gene_name": "Putative peptidyl-tRNA hydrolase PTRHD1"
}